MDM2/MDM4 family protein binding [GO:0097371] (molecular function) Definition: Binding to a member of the MDM2/MDM4 protein family, comprising negative regulators of p53. Relationships: is a type of protein binding [GO:0005515] Sources: InterPro:IPR016495